{
  "term_label": "nucleus",
  "gene_name": "B-cell lymphoma 3 protein",
  "gene_symbol": "BCL3",
  "gene": "UniProtKB:P20749",
  "term_id": "GO:0005634"
}